positive regulation of sodium-dependent phosphate transport [GO:2000120] (biological process) Sources: GOC:BHF Definition: Any process that activates or increases the frequency, rate or extent of sodium-dependent phosphate transport. Relationships: is a type of GO:0051050; is a type of GO:2000118; positively regulates sodium-dependent phosphate transport [GO:0044341]